{
  "term_label": "Unknown cellular component",
  "gene": "UniProtKB:Q9H521",
  "gene_name": "Putative uncharacterized protein LOC645739",
  "gene_symbol": "Q9H521",
  "term_id": "UNKNOWN:0003"
}